{
  "term_id": "UNKNOWN:0001",
  "term_label": "Unknown molecular function",
  "gene_symbol": "ADO",
  "gene_name": "2-aminoethanethiol dioxygenase",
  "gene": "UniProtKB:Q96SZ5"
}